superior olivary nucleus maturation [GO:0021722] (biological process) Definition: A developmental process, independent of morphogenetic (shape) change, that is required for the superior olivary nucleus to attain its fully functional state. The superior olivary nucleus is a small cylindrical mass on the dorsal surface of the lateral part of the trapezoid body of the pons, and it is situated immediately above the inferior olivary nucleus. It receives projections from the cochlear nucleus and thus is involved in the perception of sound. Sources: GOC:cls, GOC:dgh, GOC:dph, GOC:jid, GO_REF:0000021 Also known as: superior olive maturation Relationships: is a type of anatomical structure maturation [GO:0071695]; is part of pons maturation [GO:0021586]; BFO_0000050 superior olivary nucleus development [GO:0021718]